{
  "gene_name": "Cysteine desulfurase",
  "gene": "UniProtKB:Q9Y697",
  "term_label": "iron-sulfur cluster assembly",
  "term_id": "GO:0016226",
  "gene_symbol": "NFS1"
}